{
  "term_id": "GO:0005737",
  "gene_symbol": "AICDA",
  "term_label": "cytoplasm",
  "gene": "UniProtKB:Q9GZX7",
  "gene_name": "Single-stranded DNA cytosine deaminase"
}